{
  "term_label": "voltage-gated potassium channel activity",
  "gene_symbol": "LRRC52",
  "gene_name": "Leucine-rich repeat-containing protein 52",
  "term_id": "GO:0005249",
  "gene": "UniProtKB:Q8N7C0"
}